cardiolipin biosynthetic process [GO:0032049] (biological process) Sources: GOC:mah Definition: The chemical reactions and pathways resulting in the formation of cardiolipin, 1,3-bis(3-phosphatidyl)glycerol. Relationships: is_a phosphatidylglycerol biosynthetic process [GO:0006655]; is a type of cardiolipin metabolic process [GO:0032048] Also known as: diphosphatidylglycerol biosynthesis, diphosphatidylglycerol biosynthetic process